{
  "term_id": "GO:0090110",
  "gene_name": "Protein transport protein Sec24B",
  "gene_symbol": "SEC24B",
  "gene": "UniProtKB:O95487",
  "term_label": "COPII-coated vesicle cargo loading"
}